{
  "gene_symbol": "WASH6P",
  "term_label": "WASH complex",
  "gene_name": "WAS protein family homolog 6",
  "term_id": "GO:0071203",
  "gene": "UniProtKB:Q9NQA3"
}